{
  "gene_symbol": "TBPL2",
  "gene": "UniProtKB:Q6SJ96",
  "term_label": "DNA-templated transcription initiation",
  "gene_name": "TATA box-binding protein-like 2",
  "term_id": "GO:0006352"
}